{
  "gene_symbol": "TNFSF10",
  "gene": "UniProtKB:P50591",
  "gene_name": "Tumor necrosis factor ligand superfamily member 10",
  "term_label": "cell surface receptor signaling pathway",
  "term_id": "GO:0007166"
}